{
  "gene": "UniProtKB:Q92985",
  "term_label": "RNA polymerase II cis-regulatory region sequence-specific DNA binding",
  "term_id": "GO:0000978",
  "gene_name": "Interferon regulatory factor 7",
  "gene_symbol": "IRF7"
}